{
  "gene_symbol": "SF3B5",
  "term_id": "GO:0000398",
  "term_label": "mRNA splicing, via spliceosome",
  "gene_name": "Splicing factor 3B subunit 5",
  "gene": "UniProtKB:Q9BWJ5"
}